fusion of virus membrane with host macropinosome membrane [GO:0075503] (biological process) Relationships: is a type of GO:0039654 Sources: GOC:bf, GOC:jl Also known as: viral entry into host cell via macropinocytosis followed by membrane fusion with the endosome membrane, viral entry into host cell via macropinocytosis followed by membrane fusion with the host macropinosome membrane Definition: Fusion of a viral membrane with a host macropinosome membrane, that occurs after internalization of the virus through the endosomal pathway, and results in release of the viral contents into the host cell cytoplasm.